{
  "term_label": "fatty acid beta-oxidation using acyl-CoA oxidase",
  "gene": "UniProtKB:O15254",
  "gene_name": "Peroxisomal acyl-coenzyme A oxidase 3",
  "gene_symbol": "ACOX3",
  "term_id": "GO:0033540"
}